{
  "gene_symbol": "HIPK1",
  "gene_name": "Homeodomain-interacting protein kinase 1",
  "term_id": "GO:0007224",
  "term_label": "smoothened signaling pathway",
  "gene": "UniProtKB:Q86Z02"
}